torso signaling pathway [GO:0008293] (biological process) Definition: The series of molecular signals initiated by an extracellular ligand binding to torso (a receptor tyrosine kinase) on the surface of a target cell, and ending with the regulation of a downstream cellular process, e.g. transcription. References: PMID:8343949 Sources: GOC:go_curators Also known as: torso signalling pathway Relationships: is a type of cell surface receptor protein tyrosine kinase signaling pathway [GO:0007169] Regulation: regulated by GO:0120175; positively regulated by positive regulation of torso signaling pathway [GO:0120176]; negatively regulated by negative regulation of torso signaling pathway [GO:0120177]